{
  "gene": "UniProtKB:Q9P0L9",
  "term_label": "sodium channel activity",
  "gene_symbol": "PKD2L1",
  "term_id": "GO:0005272",
  "gene_name": "Polycystin-2-like protein 1"
}